{
  "gene_symbol": "TPM3",
  "term_id": "GO:0006936",
  "gene": "UniProtKB:P06753",
  "gene_name": "Tropomyosin alpha-3 chain",
  "term_label": "muscle contraction"
}